external side of mycolate outer membrane [GO:0098568] (cellular component) Definition: The side (leaflet) of the mycolate outer membrane that faces the environment and any proteins embedded in it or loosely bound to its surface. References: PMID:18316738, PMID:18567661 Sources: GOC:dos Relationships: is a type of GO:0031240